{
  "term_id": "GO:0043679",
  "gene": "UniProtKB:P30990",
  "gene_symbol": "NTS",
  "term_label": "axon terminus",
  "gene_name": "Neurotensin_neuromedin N"
}